positive regulation of axial mesodermal cell fate specification [GO:0048330] (biological process) Definition: Any process that activates or increases the frequency, rate or extent of axial mesoderm cell fate specification. Also known as: up regulation of axial mesodermal cell fate specification, up-regulation of axial mesodermal cell fate specification, upregulation of axial mesodermal cell fate specification, activation of axial mesodermal cell fate specification, stimulation of axial mesodermal cell fate specification Relationships: is a type of regulation of axial mesodermal cell fate specification [GO:0048328]; is a type of GO:0048337; positively regulates axial mesodermal cell fate specification [GO:0048327] Sources: GOC:dgh